{
  "term_id": "GO:0047291",
  "gene": "UniProtKB:Q9UNP4",
  "gene_symbol": "ST3GAL5",
  "gene_name": "Lactosylceramide alpha-2,3-sialyltransferase",
  "term_label": "lactosylceramide alpha-2,3-sialyltransferase activity"
}